{
  "gene_name": "Cardiotrophin-1",
  "term_label": "nervous system development",
  "gene": "UniProtKB:Q16619",
  "gene_symbol": "CTF1",
  "term_id": "GO:0007399"
}